alanine metabolic process [GO:0006522] (biological process) Sources: GOC:go_curators Also known as: alanine metabolism Definition: The chemical reactions and pathways involving alanine, 2-aminopropanoic acid. Subtypes: alanine biosynthetic process [GO:0006523], alanine catabolic process [GO:0006524], arginine catabolic process to alanine via ornithine [GO:0010122], L-alanine metabolic process [GO:0042851], D-alanine metabolic process [GO:0046436] Relationships: is a type of alpha-amino acid metabolic process [GO:1901605]